posterior lateral line neuromast mantle cell differentiation [GO:0048924] (biological process) Definition: The process in which a relatively unspecialized cell acquires specialized features of a posterior lateral line neuromast mantle cell. (N.B. This may be development of neuromast mantle cell type or a set of cells of neuromast mantle cell type. This will involve the change of a cell or set of cells from one cell identity to another). Mantle cells are non-sensory cells that surround the sensory strip, separating the neuromast from the epidermis. Mantle cells secrete the cupula in which the ciliary bundles of all of the hair cells are embedded. Relationships: is a type of GO:0048888; is part of GO:0048919 Sources: ISBN:0125296509